negative regulation of protein processing in phagocytic vesicle [GO:1903922] (biological process) Definition: Any process that stops, prevents or reduces the frequency, rate or extent of protein processing in phagocytic vesicle. References: PMID:23325791 Sources: GOC:TermGenie, GOC:als, GO_REF:0000058 Also known as: down regulation of protein maturation by peptide bond cleavage in phagocytic vesicle, down regulation of protein maturation by peptide bond cleavage in phagosome, down regulation of protein maturation by peptide bond hydrolysis in phagocytic vesicle, down regulation of protein maturation by peptide bond hydrolysis in phagosome, down regulation of protein processing in phagocytic vesicle, down regulation of protein processing in phagosome, down-regulation of protein maturation by peptide bond cleavage in phagocytic vesicle, down-regulation of protein maturation by peptide bond cleavage in phagosome, down-regulation of protein maturation by peptide bond hydrolysis in phagocytic vesicle, down-regulation of protein maturation by peptide bond hydrolysis in phagosome, down-regulation of protein processing in phagocytic vesicle, down-regulation of protein processing in phagosome, downregulation of protein maturation by peptide bond cleavage in phagocytic vesicle, downregulation of protein maturation by peptide bond cleavage in phagosome, downregulation of protein maturation by peptide bond hydrolysis in phagocytic vesicle, downregulation of protein maturation by peptide bond hydrolysis in phagosome, downregulation of protein processing in phagocytic vesicle, downregulation of protein processing in phagosome, negative regulation of protein maturation by peptide bond cleavage in phagocytic vesicle, negative regulation of protein maturation by peptide bond cleavage in phagosome, negative regulation of protein maturation by peptide bond hydrolysis in phagocytic vesicle, negative regulation of protein maturation by peptide bond hydrolysis in phagosome, negative regulation of protein processing in phagosome, inhibition of protein maturation by peptide bond cleavage in phagocytic vesicle, inhibition of protein maturation by peptide bond cleavage in phagosome, inhibition of protein maturation by peptide bond hydrolysis in phagocytic vesicle, inhibition of protein maturation by peptide bond hydrolysis in phagosome, inhibition of protein processing in phagocytic vesicle, inhibition of protein processing in phagosome, down regulation of peptidolysis during protein maturation in phagocytic vesicle, down regulation of peptidolysis during protein maturation in phagosome, down regulation of protein maturation by proteolysis in phagocytic vesicle, down regulation of protein maturation by proteolysis in phagosome, down-regulation of peptidolysis during protein maturation in phagocytic vesicle, down-regulation of peptidolysis during protein maturation in phagosome, down-regulation of protein maturation by proteolysis in phagocytic vesicle, down-regulation of protein maturation by proteolysis in phagosome, downregulation of peptidolysis during protein maturation in phagocytic vesicle, downregulation of peptidolysis during protein maturation in phagosome, downregulation of protein maturation by proteolysis in phagocytic vesicle, downregulation of protein maturation by proteolysis in phagosome, inhibition of peptidolysis during protein maturation in phagocytic vesicle, inhibition of peptidolysis during protein maturation in phagosome, inhibition of protein maturation by proteolysis in phagocytic vesicle, inhibition of protein maturation by proteolysis in phagosome, negative regulation of peptidolysis during protein maturation in phagocytic vesicle, negative regulation of peptidolysis during protein maturation in phagosome, negative regulation of protein maturation by proteolysis in phagocytic vesicle, negative regulation of protein maturation by proteolysis in phagosome Relationships: is a type of negative regulation of protein processing [GO:0010955]; is_a regulation of protein processing in phagocytic vesicle [GO:1903921]; negatively regulates protein processing in phagocytic vesicle [GO:1900756]